{
  "gene": "UniProtKB:Q9NPC6",
  "gene_name": "Myozenin-2",
  "term_id": "UNKNOWN:0002",
  "term_label": "Unknown biological process",
  "gene_symbol": "MYOZ2"
}